{
  "term_id": "GO:0090090",
  "gene_name": "Glycogen synthase kinase-3 alpha",
  "gene_symbol": "GSK3A",
  "term_label": "negative regulation of canonical Wnt signaling pathway",
  "gene": "UniProtKB:P49840"
}